{
  "term_id": "GO:0000139",
  "gene": "UniProtKB:Q9NY97",
  "gene_name": "N-acetyllactosaminide beta-1,3-N-acetylglucosaminyltransferase 2",
  "term_label": "Golgi membrane",
  "gene_symbol": "B3GNT2"
}